{
  "term_label": "enzyme-directed rRNA pseudouridine synthesis",
  "term_id": "GO:0000455",
  "gene": "UniProtKB:Q9UJJ7",
  "gene_name": "RNA pseudouridylate synthase domain-containing protein 1",
  "gene_symbol": "RPUSD1"
}